{
  "gene": "UniProtKB:Q92622",
  "gene_symbol": "RUBCN",
  "term_label": "negative regulation of endocytosis",
  "term_id": "GO:0045806",
  "gene_name": "Run domain Beclin-1-interacting and cysteine-rich domain-containing protein"
}